{
  "gene": "UniProtKB:Q96DB5",
  "term_id": "GO:0005737",
  "term_label": "cytoplasm",
  "gene_symbol": "RMDN1",
  "gene_name": "Regulator of microtubule dynamics protein 1"
}